{
  "term_label": "5'-3' DNA helicase activity",
  "gene_symbol": "PIF1",
  "term_id": "GO:0043139",
  "gene": "UniProtKB:Q9H611",
  "gene_name": "ATP-dependent DNA helicase PIF1"
}